{
  "gene_name": "S1 RNA-binding domain-containing protein 1",
  "term_id": "UNKNOWN:0003",
  "term_label": "Unknown cellular component",
  "gene": "UniProtKB:Q8N5C6",
  "gene_symbol": "SRBD1"
}